{
  "gene_name": "Rhotekin",
  "gene_symbol": "RTKN",
  "gene": "UniProtKB:Q9BST9",
  "term_id": "GO:0031106",
  "term_label": "septin ring organization"
}